host-mediated modulation of intestinal microbiota composition [GO:0048874] (biological process) Relationships: is a type of GO:0048872; is a type of host-mediated perturbation of symbiont process [GO:0051851] References: PMID:25757720 Definition: The biological process involved in maintaining the steady-state number of cells within a population of free-living cells such as the bacteria in the gut. Also known as: host-mediated regulation of intestinal microbiota composition, homeostasis of number of cells in a free-living population, host-induced regulation of intestinal microbiota composition